ecdysone 20-monooxygenase activity [GO:0004501] (molecular function) Definition: Catalysis of the reaction: AH(2) + ecdysone + O2 = 20-hydroxyecdysone + A + H2O. Sources: EC:1.14.99.22, RHEA:14021 Relationships: is a type of steroid hydroxylase activity [GO:0008395]; is a type of oxidoreductase activity, acting on paired donors, with incorporation or reduction of molecular oxygen [GO:0016705] Also known as: ecdysone modification, ecdysone 20-hydroxylase activity, alpha-ecdysone C-20 hydroxylase activity, ecdysone,hydrogen-donor:oxygen oxidoreductase (20-hydroxylating)